intermediate-density lipoprotein particle clearance [GO:0071831] (biological process) Definition: The process in which a intermediate-density lipoprotein particle is removed from the blood via receptor-mediated endocytosis and its constituent parts degraded. Sources: GOC:BHF Also known as: IDL clearance Relationships: is a type of triglyceride-rich lipoprotein particle clearance [GO:0071830]